{
  "term_label": "negative regulation of cAMP/PKA signal transduction",
  "term_id": "GO:0141162",
  "gene": "UniProtKB:P51160",
  "gene_symbol": "PDE6C",
  "gene_name": "Cone cGMP-specific 3',5'-cyclic phosphodiesterase subunit alpha'"
}